protein localization to postsynaptic specialization membrane [GO:0099633] (biological process) Definition: A process in which a protein is transported to, or maintained in, a location within the membrane adjacent to a postsynaptic specialization (e.g. post synaptic density). Sources: GOC:dos Also known as: protein localisation in postsynaptic specialization membrane Relationships: is a type of protein localization to organelle [GO:0033365]; is a type of protein localization to postsynaptic membrane [GO:1903539] Subtypes: neurotransmitter receptor localization to postsynaptic specialization membrane [GO:0099645]